{
  "term_id": "GO:0015677",
  "term_label": "copper ion import",
  "gene_name": "Metalloreductase STEAP4",
  "gene_symbol": "STEAP4",
  "gene": "UniProtKB:Q687X5"
}